{
  "gene": "UniProtKB:Q8N441",
  "gene_symbol": "FGFRL1",
  "gene_name": "Fibroblast growth factor receptor-like 1",
  "term_label": "plasma membrane",
  "term_id": "GO:0005886"
}